phospholipase C-inhibiting G protein-coupled receptor signaling pathway [GO:0030845] (biological process) References: PMID:8280098 Sources: GOC:dph, GOC:mah, GOC:signaling, GOC:tb Definition: A G protein-coupled receptor signaling pathway which proceeds with inhibition of phospholipase C (PLC) activity and a subsequent decrease in the levels of cellular inositol trisphosphate (IP3) and diacylglycerol (DAG). Also known as: G-protein-coupled inhibitory pathway of phospholipase C, GPCR signaling pathway coupled to inhibition of phospholipase C activity, GPCR signaling pathway via inhibition of PLC, PLC-inhibiting GPCR signaling pathway, phospholipase C-inhibiting G-protein coupled receptor signaling pathway, inhibition of phospholipase C activity involved in G-protein coupled receptor signalling pathway, phospholipase C inhibition Relationships: is a type of G protein-coupled receptor signaling pathway [GO:0007186]; has part phospholipase C inhibitor activity [GO:0160186] Note: This term is intended to cover steps in a GPCR signaling pathway both upstream and downstream of phospholipase C (PLC) inhibition.